hydroxyquinol 1,2-dioxygenase activity [GO:0018581] (molecular function) Sources: RHEA:19441 Definition: Catalysis of the reaction: benzene-1,2,4-triol + O2 = 3-hydroxy-cis,cis-muconate + 2 H+. Relationships: is a type of oxidoreductase activity, acting on single donors with incorporation of molecular oxygen, incorporation of two atoms of oxygen [GO:0016702]